cardiolipin synthase (CMP-forming) [GO:0043337] (molecular function) Also known as: cardiolipin synthase, cardiolipin synthetase, CDP-diacylglycerol-phosphatidylglycerol phosphatidyltransferase activity Sources: GOC:jl Relationships: is a type of phosphatidyltransferase activity [GO:0030572] Definition: Catalysis of the reaction: CDP-diacylglycerol + phosphatidylglycerol = CMP + diphosphatidylglycerol.